negative regulation of interleukin-4 production [GO:0032713] (biological process) Also known as: down regulation of interleukin-4 production, down-regulation of interleukin-4 production, downregulation of interleukin-4 production, negative regulation of IL-4 production, inhibition of interleukin-4 production, negative regulation of interleukin-4 biosynthetic process, negative regulation of interleukin-4 secretion References: PMID:29778524 Sources: GOC:mah Relationships: is a type of GO:0001818; is_a regulation of interleukin-4 production [GO:0032673]; negatively regulates interleukin-4 production [GO:0032633] Definition: Any process that stops, prevents, or reduces the frequency, rate, or extent of interleukin-4 production.